myo-inositol hexakisphosphate biosynthetic process, lipid-independent [GO:0033548] (biological process) Definition: The chemical reactions and pathways resulting in the formation of phytic acid, myo-inositol hexakisphosphate, by the successively phosphorylation of myo-inositol or an inositol trisphosphate; the inositol trisphosphates that may be used by this pathway are inositol 3,4,5-trisphosphate and inositol 3,4,6trisphosphate. Also known as: myo-inositol hexakisphosphate anabolism, lipid-independent, myo-inositol hexakisphosphate biosynthesis, lipid-independent, myo-inositol hexakisphosphate formation, lipid-independent, myo-inositol hexakisphosphate synthesis, lipid-independent, phytate biosynthesis, lipid-independent, phytate biosynthetic process, lipid-independent Relationships: is a type of myo-inositol hexakisphosphate biosynthetic process [GO:0010264] Sources: GOC:mah, MetaCyc:PWY-4661